amyloid-beta clearance by transcytosis [GO:0150093] (biological process) References: PMID:26005850 Sources: GOC:aruk, GOC:bc Definition: The process in which amyloid-beta is removed from extracellular brain regions by cell surface receptor-mediated endocytosis, followed by transcytosis across the blood-brain barrier. Relationships: is a type of transcytosis [GO:0045056]; is a type of amyloid-beta clearance [GO:0097242]